{
  "term_label": "apoptotic DNA fragmentation",
  "gene_symbol": "DICER1",
  "term_id": "GO:0006309",
  "gene_name": "Endoribonuclease Dicer",
  "gene": "UniProtKB:Q9UPY3"
}